{
  "gene_symbol": "H1-1",
  "gene": "UniProtKB:Q02539",
  "gene_name": "Histone H1.1",
  "term_label": "spermatogenesis",
  "term_id": "GO:0007283"
}